{
  "gene": "UniProtKB:Q4LE39",
  "term_label": "regulation of transcription by RNA polymerase II",
  "gene_symbol": "ARID4B",
  "term_id": "GO:0006357",
  "gene_name": "AT-rich interactive domain-containing protein 4B"
}